berbamunine synthase activity [GO:0047054] (molecular function) Sources: RHEA:23576 Relationships: is a type of oxidoreductase activity, acting on paired donors, with oxidation of a pair of donors resulting in the reduction of molecular oxygen to two molecules of water [GO:0016717] Definition: Catalysis of the reaction: (S)-N-methylcoclaurine + (R)-N-methylcoclaurine + [reduced NADPH--hemoprotein reductase] + O2 = berbamunine + [oxidized NADPH--hemoprotein reductase] + 2 H2O. Also known as: heme-thiolate